RNA adenosine-uridine insertion [GO:0070711] (biological process) Sources: GOC:cb, GOC:mah Definition: The modification of an RNA molecule by insertion of an adenosine-uridine dinucleotide. Also known as: RNA AU insertion Relationships: is a type of RNA dinucleotide insertion [GO:0070707]